{
  "gene_name": "RING finger protein 207",
  "term_id": "GO:1901207",
  "term_label": "regulation of heart looping",
  "gene_symbol": "RNF207",
  "gene": "UniProtKB:Q6ZRF8"
}